{
  "term_id": "GO:0004715",
  "gene_name": "Tyrosine-protein kinase FRK",
  "gene": "UniProtKB:P42685",
  "gene_symbol": "FRK",
  "term_label": "non-membrane spanning protein tyrosine kinase activity"
}